{
  "gene": "UniProtKB:Q9UKL0",
  "gene_name": "REST corepressor 1",
  "gene_symbol": "RCOR1",
  "term_label": "regulation of transcription by RNA polymerase II",
  "term_id": "GO:0006357"
}